regulation of cardiocyte differentiation [GO:1905207] (biological process) Definition: Any process that modulates the frequency, rate or extent of cardiocyte differentiation. Relationships: is a type of GO:0045595; regulates GO:0035051 References: PMID:23069713 Sources: GOC:BHF, GOC:BHF_miRNA, GOC:TermGenie, GOC:bc, GO_REF:0000058 Subtypes: regulation of cardioblast differentiation [GO:0051890], GO:0120074, negative regulation of cardiocyte differentiation [GO:1905208], positive regulation of cardiocyte differentiation [GO:1905209], regulation of cardiac cell fate specification [GO:2000043], regulation of cardiac vascular smooth muscle cell differentiation [GO:2000722], regulation of cardiac muscle cell differentiation [GO:2000725] Also known as: regulation of cardiac cell differentiation, regulation of heart cell differentiation